glucomannan metabolic process [GO:0010391] (biological process) Definition: The chemical reactions and pathways involving glucomannan, a polysaccharide composed of D-glucose and D-mannose. The mannose units form the backbone structure (a linear main chain) with the D-glucose as single side-units. Subtypes: glucomannan catabolic process [GO:2000884] Also known as: glucomannan metabolism Sources: GOC:tair_curators Relationships: is a type of substituted mannan metabolic process [GO:0006080]